{
  "term_label": "regulation of cell motility",
  "gene": "UniProtKB:Q6ZS72",
  "gene_name": "Protein PEAK3",
  "gene_symbol": "PEAK3",
  "term_id": "GO:2000145"
}